gamma-1,2,3,4,5,6-hexachlorocyclohexane metabolic process [GO:0018919] (biological process) Definition: The chemical reactions and pathways involving gamma-1,2,3,4,5,6-hexachlorocyclohexane (also known as Lindane), the most common form of hexachlorohexane, a halogenated organic insecticide that has been used worldwide for agriculture and public health. Also known as: gamma-1,2,3,4,5,6-hexachlorocyclohexane metabolism Relationships: is a type of hexachlorocyclohexane metabolic process [GO:0019497] Sources: UM-BBD_pathwayID:ghch